{
  "gene": "UniProtKB:P24864",
  "gene_name": "G1_S-specific cyclin-E1",
  "term_label": "positive regulation of G1/S transition of mitotic cell cycle",
  "term_id": "GO:1900087",
  "gene_symbol": "CCNE1"
}